{
  "gene": "UniProtKB:Q5BKX5",
  "gene_name": "Actin maturation protease",
  "gene_symbol": "ACTMAP",
  "term_label": "Unknown biological process",
  "term_id": "UNKNOWN:0002"
}